termination of monopolar cell growth [GO:0051521] (biological process) Definition: Any process that stops the active process of bipolar cell growth, polarized growth from one end of a cell. Sources: GOC:ai Relationships: is a type of negative regulation of monopolar cell growth [GO:0051514]